{
  "term_label": "Golgi stack",
  "term_id": "GO:0005795",
  "gene": "UniProtKB:Q9UM21",
  "gene_name": "Alpha-1,3-mannosyl-glycoprotein 4-beta-N-acetylglucosaminyltransferase A",
  "gene_symbol": "MGAT4A"
}